{
  "term_label": "endoplasmic reticulum",
  "gene_symbol": "STIM2",
  "term_id": "GO:0005783",
  "gene_name": "Stromal interaction molecule 2",
  "gene": "UniProtKB:Q9P246"
}